ligand-gated sodium channel activity [GO:0015280] (molecular function) Definition: Enables the transmembrane transfer of a sodium ion by a channel that opens when a specific ligand has been bound by the channel complex or one of its constituent parts. Subtypes: kainate selective glutamate receptor activity [GO:0015277], GO:0160125 Relationships: is a type of sodium channel activity [GO:0005272]; is_a ligand-gated monoatomic cation channel activity [GO:0099094] Sources: GOC:mah Also known as: acid-sensing ion channel activity, epithelial sodium channel